negative regulation of translational frameshifting [GO:2001125] (biological process) Relationships: is a type of negative regulation of translational elongation [GO:0045900]; is a type of regulation of translational frameshifting [GO:2001124]; negatively regulates translational frameshifting [GO:0006452] Definition: Any process that stops, prevents or reduces the frequency, rate or extent of translational frameshifting. Sources: GOC:obol